negative regulation of calcineurin-NFAT signaling cascade [GO:0070885] (BP) Also known as: down regulation of calcineurin-NFAT signaling cascade, down-regulation of calcineurin-NFAT signaling cascade, downregulation of calcineurin-NFAT signaling cascade, negative regulation of calcineurin-NFAT signalling cascade, inhibition of NFAT protein import into nucleus, inhibition of calcineurin-NFAT signaling cascade, negative regulation of NFAT protein import into nucleus, termination of calcineurin-NFAT signaling cascade, negative regulation of calcineurin-NFAT signaling pathway Sources: GOC:mah Relationships: is a type of regulation of calcineurin-NFAT signaling cascade [GO:0070884]; is a type of negative regulation of calcineurin-mediated signaling [GO:0106057]; RO_0002212 calcineurin-NFAT signaling cascade [GO:0033173] Definition: Any process that stops, prevents, or reduces the frequency, rate or extent of the calcineurin-NFAT signaling cascade.